{
  "gene": "UniProtKB:Q9Y225",
  "term_id": "UNKNOWN:0002",
  "gene_symbol": "RNF24",
  "term_label": "Unknown biological process",
  "gene_name": "RING finger protein 24"
}